{
  "term_label": "PR-DUB complex",
  "gene": "UniProtKB:Q8IXJ9",
  "gene_name": "Polycomb group protein ASXL1",
  "gene_symbol": "ASXL1",
  "term_id": "GO:0035517"
}